chrysobactin catabolic process [GO:0042859] (biological process) Definition: The chemical reactions and pathways resulting in the breakdown of the siderophore chrysobactin (alpha-N-(2,3-dihydroxybenzoyl)-D-lysyl-L-serine). Also known as: chrysobactin breakdown, chrysobactin catabolism, chrysobactin degradation References: PMID:8837459 Sources: GOC:jl Relationships: is a type of GO:0019614; is_a GO:0034310; is a type of amide metabolic process [GO:0043603]; is_a siderophore catabolic process [GO:0046215]; is a type of carboxylic acid catabolic process [GO:0046395]; is a type of primary amino compound catabolic process [GO:1901161]